mitochondrial glutaminyl-tRNA aminoacylation [GO:0070148] (biological process) Definition: The process of coupling glutamine to glutaminyl-tRNA in a mitochondrion, catalyzed by glutaminyl-tRNA synthetase. In tRNA aminoacylation, the amino acid is first activated by linkage to AMP and then transferred to either the 2'- or the 3'-hydroxyl group of the 3'-adenosine residue of the tRNA. Sources: GOC:mah, GOC:mcc Relationships: is a type of glutaminyl-tRNA aminoacylation [GO:0006425]; is a type of GO:0070127